post-mRNA release spliceosomal complex [GO:0071014] (cellular component) Relationships: is a type of GO:0005681; has part GO:0005682 Subtypes: U2-type post-mRNA release spliceosomal complex [GO:0071008], U12-type post-mRNA release spliceosomal complex [GO:0071019] References: PMID:19239890, PMID:20149226 Sources: GOC:ab, GOC:krc, GOC:mah, ISBN:0879695897 Definition: A spliceosomal complex that is formed following the release of the spliced product from the post-spliceosomal complex and contains the excised intron and three snRNPs, either U2 or U12, U5, and either U6 or U6atac. Also known as: mammalian spliceosomal complex I